{
  "term_label": "Unknown molecular function",
  "gene": "UniProtKB:Q6W0C5",
  "gene_name": "Developmental pluripotency-associated protein 3",
  "gene_symbol": "DPPA3",
  "term_id": "UNKNOWN:0001"
}